{
  "gene_name": "E3 ubiquitin-protein ligase RFWD3",
  "gene_symbol": "RFWD3",
  "gene": "UniProtKB:Q6PCD5",
  "term_id": "GO:0005634",
  "term_label": "nucleus"
}